{
  "gene_name": "Protein PAT1 homolog 1",
  "term_id": "GO:0003723",
  "gene_symbol": "PATL1",
  "gene": "UniProtKB:Q86TB9",
  "term_label": "RNA binding"
}